{
  "gene_symbol": "SPC25",
  "gene": "UniProtKB:Q9HBM1",
  "term_label": "chromosome segregation",
  "term_id": "GO:0007059",
  "gene_name": "Kinetochore protein Spc25"
}